{
  "term_label": "signal transduction",
  "gene_symbol": "CAMKV",
  "gene_name": "CaM kinase-like vesicle-associated protein",
  "gene": "UniProtKB:Q8NCB2",
  "term_id": "GO:0007165"
}